{
  "gene_name": "Serine_threonine-protein phosphatase 2A 56 kDa regulatory subunit gamma isoform",
  "gene": "UniProtKB:Q13362",
  "gene_symbol": "PPP2R5C",
  "term_id": "GO:0000159",
  "term_label": "protein phosphatase type 2A complex"
}